{
  "gene_symbol": "PAPPA",
  "term_id": "GO:0005615",
  "gene": "UniProtKB:Q13219",
  "gene_name": "Pappalysin-1",
  "term_label": "extracellular space"
}